regulation of circadian sleep/wake cycle, non-REM sleep [GO:0045188] (biological process) Definition: Any process that modulates the frequency, rate or extent of non-rapid eye movement sleep. Sources: GOC:go_curators Also known as: regulation of non-REM sleep Relationships: is a type of regulation of circadian sleep/wake cycle, sleep [GO:0045187]; regulates GO:0042748 Subtypes: negative regulation of circadian sleep/wake cycle, non-REM sleep [GO:0042323], positive regulation of circadian sleep/wake cycle, non-REM sleep [GO:0046010]